cyanidin-3-rhamnosylglucoside 5-O-glucosyltransferase activity [GO:0047214] (molecular function) Sources: EC:2.4.1.116, MetaCyc:2.4.1.116-RXN Also known as: UDP-glucose:cyanidin-3-O-D-rhamnosyl-1,6-D-glucoside 5-O-D-glucosyltransferase activity, UDP-glucose:cyanidin-3-O-beta-L-rhamnosyl-(1->6)-beta-D-glucoside 5-O-beta-D-glucosyltransferase activity, cyanidin-3-O-rutinoside 5-O-glucosyltransferase activity, uridine diphosphoglucose-cyanidin 3-rhamnosylglucoside 5-O-glucosyltransferase activity Definition: Catalysis of the reaction: cyanidin-3-O-D-rhamnosyl-(1,6)-D-glucoside + UDP-D-glucose = cyanidin-3-O-[D-rhamnosyl-(1,6)-D-glucoside]-5-O-D-glucoside + UDP. Relationships: is a type of UDP-glucosyltransferase activity [GO:0035251]